{
  "gene": "UniProtKB:O60861",
  "term_label": "plasma membrane",
  "gene_symbol": "GAS7",
  "gene_name": "Growth arrest-specific protein 7",
  "term_id": "GO:0005886"
}